{
  "term_label": "synaptic membrane",
  "term_id": "GO:0097060",
  "gene_symbol": "PALM",
  "gene_name": "Paralemmin-1",
  "gene": "UniProtKB:O75781"
}